regulation of anterior/posterior axon guidance [GO:1905486] (biological process) Definition: Any process that modulates the frequency, rate or extent of anterior/posterior axon guidance. Relationships: is a type of regulation of axon guidance [GO:1902667]; regulates anterior/posterior axon guidance [GO:0033564] Also known as: regulation of anterior-posterior axon guidance, regulation of anterior/posterior axon pathfinding Subtypes: negative regulation of anterior/posterior axon guidance [GO:1905487], positive regulation of anterior/posterior axon guidance [GO:1905488] References: PMID:16516839 Sources: GOC:TermGenie, GO_REF:0000058